floral organ abscission [GO:0010227] (biological process) Regulation: regulated by regulation of floral organ abscission [GO:0060860]; positively regulated by positive regulation of floral organ abscission [GO:0060861]; negatively regulated by negative regulation of floral organ abscission [GO:0060862] Relationships: is a type of developmental process involved in reproduction [GO:0003006]; is a type of GO:0009838; BFO_0000050 floral organ development [GO:0048437] Definition: The controlled shedding of floral organs. References: PMID:12972671 Sources: GOC:PO_curators, PO:0025395